{
  "gene": "UniProtKB:Q5K4L6",
  "term_id": "GO:0005739",
  "gene_name": "Long-chain fatty acid transport protein 3",
  "term_label": "mitochondrion",
  "gene_symbol": "SLC27A3"
}